regulation of leukocyte adhesion to arterial endothelial cell [GO:1904997] (BP) Relationships: is a type of regulation of leukocyte adhesion to vascular endothelial cell [GO:1904994]; regulates leukocyte adhesion to arterial endothelial cell [GO:0061757] References: PMID:22267480 Sources: GOC:BHF, GOC:BHF_miRNA, GOC:TermGenie, GOC:bc, GO_REF:0000058 Subtypes: negative regulation of leukocyte adhesion to arterial endothelial cell [GO:1904998], positive regulation of leukocyte adhesion to arterial endothelial cell [GO:1904999] Definition: Any process that modulates the frequency, rate or extent of leukocyte adhesion to arterial endothelial cell.